{
  "term_label": "innate immune response",
  "gene": "UniProtKB:Q495X7",
  "gene_symbol": "TRIM60",
  "term_id": "GO:0045087",
  "gene_name": "Tripartite motif-containing protein 60"
}